{
  "gene_name": "Breast cancer type 1 susceptibility protein",
  "term_id": "GO:0045944",
  "gene_symbol": "BRCA1",
  "term_label": "positive regulation of transcription by RNA polymerase II",
  "gene": "UniProtKB:P38398"
}